cardiac myofibril assembly [GO:0055003] (biological process) Sources: GOC:devbiol Also known as: cardiac myofibril development, cardiac myofibril morphogenesis, heart myofibril assembly Regulation: regulated by regulation of cardiac myofibril assembly [GO:1905304]; negatively regulated by GO:1905305; positively regulated by positive regulation of cardiac myofibril assembly [GO:1905306] Subtypes: atrial cardiac myofibril assembly [GO:0055004], GO:0055005 Definition: The process whose specific outcome is the progression of the cardiac myofibril over time, from its formation to the mature structure. A cardiac myofibril is a myofibril specific to cardiac muscle cells. Relationships: is a type of myofibril assembly [GO:0030239]; is part of cardiac muscle cell development [GO:0055013]